{
  "term_id": "GO:0045030",
  "gene_symbol": "P2RY2",
  "gene": "UniProtKB:P41231",
  "gene_name": "P2Y purinoceptor 2",
  "term_label": "G protein-coupled UTP receptor activity"
}